{
  "gene_symbol": "PTP4A3",
  "term_label": "cytoplasm",
  "term_id": "GO:0005737",
  "gene": "UniProtKB:O75365",
  "gene_name": "Protein tyrosine phosphatase type IVA 3"
}